nitric oxide dioxygenase activity, heme protein as donor [GO:0141118] (MF) Relationships: is a type of oxidoreductase activity, acting on a heme group of donors [GO:0016675] Definition: Catalysis of the reaction: Fe(II)-heme b-[protein] + nitric oxide + O2 = Fe(III)-heme b-[protein] + nitrate. References: PMID:20511233 Note: Note that this activity is similar to nitric oxide dioxygenase activity ; GO:0008941, but GO:000894 uses NADPH as the electron donor.